hydroxypyruvate reductase (NADH) activity [GO:0008465] (molecular function) Sources: EC:1.1.1.29 Also known as: glycerate dehydrogenase activity, hydroxypyruvate dehydrogenase activity, glycerate dehydrogenase (NAD+) activity Relationships: is a type of hydroxypyruvate reductase [NAD(P)H] activity [GO:0016618] Definition: Catalysis of the reaction: (R)-glycerate + NAD+ = 3-hydroxypyruvate + NADH + H+.